preprotein binding [GO:0070678] (molecular function) Definition: Binding to a preprotein, the unprocessed form of a protein destined to undergo co- or post-translational processing. References: PMID:12914940 Sources: GOC:imk, GOC:mah Also known as: unprocessed protein binding Relationships: is a type of protein binding [GO:0005515]